{
  "gene_name": "Potassium voltage-gated channel subfamily E member 3",
  "gene": "UniProtKB:Q9Y6H6",
  "term_label": "regulation of ventricular cardiac muscle cell membrane repolarization",
  "term_id": "GO:0060307",
  "gene_symbol": "KCNE3"
}